{
  "gene_symbol": "CYBC1",
  "gene": "UniProtKB:Q9BQA9",
  "term_id": "UNKNOWN:0001",
  "term_label": "Unknown molecular function",
  "gene_name": "Cytochrome b-245 chaperone 1"
}